{
  "gene": "UniProtKB:Q9HBH0",
  "term_label": "GTPase activity",
  "gene_name": "Rho-related GTP-binding protein RhoF",
  "gene_symbol": "RHOF",
  "term_id": "GO:0003924"
}